{
  "gene_symbol": "H2BC18",
  "gene": "UniProtKB:Q5QNW6",
  "term_label": "nucleus",
  "term_id": "GO:0005634",
  "gene_name": "Histone H2B type 2-F"
}